{
  "term_label": "cis-Golgi network",
  "gene_name": "ER lumen protein-retaining receptor 1",
  "gene": "UniProtKB:P24390",
  "term_id": "GO:0005801",
  "gene_symbol": "KDELR1"
}